{
  "term_id": "GO:1990904",
  "gene": "UniProtKB:Q15434",
  "term_label": "ribonucleoprotein complex",
  "gene_symbol": "RBMS2",
  "gene_name": "RNA-binding motif, single-stranded-interacting protein 2"
}